rRNA (pseudouridine-N3-)-methyltransferase activity [GO:0070038] (molecular function) Sources: GOC:imk, GOC:mah Relationships: is a type of rRNA (pseudouridine) methyltransferase activity [GO:0070037] Definition: Catalysis of the reaction: S-adenosyl-L-methionine + rRNA = S-adenosyl-L-homocysteine + rRNA containing N3-methylpseudouridine.